{
  "gene_name": "Muscarinic acetylcholine receptor M2",
  "term_id": "GO:0007187",
  "gene": "UniProtKB:P08172",
  "gene_symbol": "CHRM2",
  "term_label": "G protein-coupled receptor signaling pathway, coupled to cyclic nucleotide second messenger"
}